aculeacin-A deacylase activity [GO:0033965] (molecular function) Also known as: aculeacin A acylase activity, aculeacin-A amidohydrolase activity Relationships: is_a GO:0016811 Sources: EC:3.5.1.70 Definition: Catalysis of the hydrolysis of the amide bond in aculeacin A and related neutral lipopeptide antibiotics, releasing the long-chain fatty acid side-chain.